{
  "gene_name": "Olfactory receptor 5H2",
  "term_label": "olfactory receptor activity",
  "gene_symbol": "OR5H2",
  "term_id": "GO:0004984",
  "gene": "UniProtKB:Q8NGV7"
}